extrinsic component of synaptic vesicle membrane [GO:0098850] (cellular component) Relationships: is a type of extrinsic component of organelle membrane [GO:0031312]; BFO_0000050 synaptic vesicle membrane [GO:0030672] Sources: GOC:dos Definition: The component of the synaptic vesicle membrane consisting of gene products and protein complexes that are loosely bound to one of its surfaces, but not integrated into the hydrophobic region.